bile acid secretion [GO:0032782] (biological process) Relationships: is_a monocarboxylic acid transport [GO:0015718]; is a type of acid secretion [GO:0046717] Definition: The regulated release of bile acid, composed of any of a group of steroid carboxylic acids occurring in bile, by a cell or a tissue. Regulation: regulated by regulation of bile acid secretion [GO:0120188]; positively regulated by GO:0120189; negatively regulated by negative regulation of bile acid secretion [GO:0120190] Sources: GOC:ecd